{
  "gene": "UniProtKB:Q96L21",
  "term_id": "GO:0006412",
  "gene_name": "Ribosomal protein uL16-like",
  "gene_symbol": "RPL10L",
  "term_label": "translation"
}